regulation of interleukin-3 production [GO:0032672] (biological process) Definition: Any process that modulates the frequency, rate, or extent of interleukin-3 production. Subtypes: negative regulation of interleukin-3 production [GO:0032712], GO:0032752 Sources: GOC:mah Also known as: regulation of IL-3 production, regulation of interleukin-3 biosynthetic process Relationships: is a type of regulation of cytokine production [GO:0001817]; regulates GO:0032632